{
  "term_label": "axon",
  "gene_symbol": "POTEJ",
  "term_id": "GO:0030424",
  "gene": "UniProtKB:P0CG39",
  "gene_name": "POTE ankyrin domain family member J"
}